propanediol-phosphate dehydrogenase activity [GO:0050216] (molecular function) Sources: EC:1.1.1.7, RHEA:21584 Definition: Catalysis of the reaction: NAD+ + propane-1,2-diol 1-phosphate = H+ + hydroxyacetone phosphate + NADH. Relationships: is a type of oxidoreductase activity, acting on the CH-OH group of donors, NAD or NADP as acceptor [GO:0016616]